{
  "term_id": "GO:0003924",
  "term_label": "GTPase activity",
  "gene_name": "Rab-like protein 2A",
  "gene": "UniProtKB:Q9UBK7",
  "gene_symbol": "RABL2A"
}